{
  "gene": "UniProtKB:Q6ZNX1",
  "term_label": "Unknown molecular function",
  "gene_symbol": "SHLD3",
  "gene_name": "Shieldin complex subunit 3",
  "term_id": "UNKNOWN:0001"
}